cellular response to bismuth [GO:0072701] (biological process) Definition: Any process that results in a change in state or activity of a cell (in terms of movement, secretion, enzyme production, gene expression, etc.) as a result of a bismuth (Bi) stimulus. Sources: GOC:mah Also known as: cellular response to bismuth ion Relationships: is a type of cellular response to chemical stimulus [GO:0070887]; is a type of response to bismuth [GO:0072700]